{
  "gene_name": "Histidine-rich glycoprotein",
  "term_label": "positive regulation of immune response to tumor cell",
  "gene": "UniProtKB:P04196",
  "term_id": "GO:0002839",
  "gene_symbol": "HRG"
}